provirus excision [GO:0032359] (biological process) Also known as: prophage excision Relationships: is a type of GO:0019046 Definition: The molecular events that lead to the excision of a viral genome from the host genome. Sources: GOC:mlg, VZ:3969